{
  "term_label": "nucleus",
  "term_id": "GO:0005634",
  "gene_name": "Nuclear body protein SP140",
  "gene": "UniProtKB:Q13342",
  "gene_symbol": "SP140"
}